{
  "gene_symbol": "CAMLG",
  "gene_name": "Guided entry of tail-anchored proteins factor CAMLG",
  "term_id": "GO:0071816",
  "gene": "UniProtKB:P49069",
  "term_label": "tail-anchored membrane protein insertion into ER membrane"
}